5-amino-6-(D-ribitylamino)uracil--L-tyrosine 4-hydroxyphenyl transferase activity [GO:0141093] (molecular function) References: PMID:11948155, PMID:23072415, PMID:25781338 Sources: RHEA:55200 Definition: Catalysis of the reaction: 5-amino-6-(D-ribitylamino)uracil + L-tyrosine + S-adenosyl-L-methionine = 2-iminoacetate + 5'-deoxyadenosine + 5-amino-5-(4-hydroxybenzyl)-6-(D-ribitylimino)-5,6-dihydrouracil + H+ + L-methionine. Relationships: is a type of transferase activity, transferring alkyl or aryl (other than methyl) groups [GO:0016765]